tubulin N-terminal-methionine acetyltransferase activity [GO:0120519] (molecular function) Definition: Catalysis of the reaction: acetyl-CoA + N-terminal L-methionyl-[tubulin] = CoA + H+ + N-terminal N(alpha)-acetyl-L-methionyl-[tubulin]. The N-terminus of both alpha- and beta-tubulin are acetylated. Sources: EC:2.3.1.308, RHEA:69607 Also known as: tubulin N-terminal N-acetyltransferase activity Relationships: is a type of GO:0004596